{
  "term_label": "calmodulin binding",
  "gene": "UniProtKB:Q13555",
  "gene_symbol": "CAMK2G",
  "gene_name": "Calcium_calmodulin-dependent protein kinase type II subunit gamma",
  "term_id": "GO:0005516"
}